negative regulation of immunoglobulin mediated immune response [GO:0002890] (biological process) Definition: Any process that stops, prevents, or reduces the frequency, rate, or extent of an immunoglobulin mediated immune response. Sources: GOC:add Also known as: down regulation of immunoglobulin mediated immune response, down-regulation of immunoglobulin mediated immune response, downregulation of immunoglobulin mediated immune response, inhibition of immunoglobulin mediated immune response Relationships: is a type of negative regulation of B cell mediated immunity [GO:0002713]; is_a regulation of immunoglobulin mediated immune response [GO:0002889]; RO_0002212 immunoglobulin mediated immune response [GO:0016064] Subtypes: negative regulation of type III hypersensitivity [GO:0001804], negative regulation of type I hypersensitivity [GO:0001811], negative regulation of type II hypersensitivity [GO:0002893], negative regulation of humoral immune response mediated by circulating immunoglobulin [GO:0002924], negative regulation of isotype switching [GO:0045829]